sperm head plasma membrane [GO:1990913] (cellular component) Definition: The plasma membrane that is part of the head section of a sperm cell. References: PMID:24478030 Relationships: is a type of plasma membrane region [GO:0098590]; BFO_0000050 sperm head [GO:0061827]; is part of GO:0097524